{
  "gene_name": "Toll-like receptor 4",
  "term_label": "MyD88-dependent toll-like receptor signaling pathway",
  "gene_symbol": "TLR4",
  "gene": "UniProtKB:O00206",
  "term_id": "GO:0002755"
}